{
  "gene_name": "Palmitoleoyl-protein carboxylesterase NOTUM",
  "term_label": "Unknown cellular component",
  "term_id": "UNKNOWN:0003",
  "gene": "UniProtKB:Q6P988",
  "gene_symbol": "NOTUM"
}